{
  "term_label": "growth factor binding",
  "gene": "UniProtKB:P35916",
  "term_id": "GO:0019838",
  "gene_name": "Vascular endothelial growth factor receptor 3",
  "gene_symbol": "FLT4"
}